{
  "gene_symbol": "KCNJ11",
  "term_id": "GO:0005242",
  "term_label": "inward rectifier potassium channel activity",
  "gene_name": "ATP-sensitive inward rectifier potassium channel 11",
  "gene": "UniProtKB:Q14654"
}